{
  "gene": "UniProtKB:Q9Y3P9",
  "term_id": "UNKNOWN:0002",
  "gene_name": "Rab GTPase-activating protein 1",
  "gene_symbol": "RABGAP1",
  "term_label": "Unknown biological process"
}